ectodermal cell differentiation [GO:0010668] (biological process) Sources: GOC:dph, GOC:tb Relationships: is_a cell differentiation [GO:0030154]; is part of ectoderm development [GO:0007398] Definition: The process in which relatively unspecialized cells acquire specialized structural and/or functional features of an ectodermal cell. Differentiation includes the processes involved in commitment of a cell to a specific fate.